{
  "gene": "UniProtKB:O14734",
  "term_label": "acyl-CoA metabolic process",
  "term_id": "GO:0006637",
  "gene_name": "Acyl-coenzyme A thioesterase 8",
  "gene_symbol": "ACOT8"
}